{
  "term_label": "glycerophospholipid biosynthetic process",
  "gene_symbol": "HDHD5",
  "term_id": "GO:0046474",
  "gene_name": "Haloacid dehalogenase-like hydrolase domain-containing 5",
  "gene": "UniProtKB:Q9BXW7"
}